{
  "gene_name": "Iron-sulfur cluster co-chaperone protein HscB",
  "term_id": "UNKNOWN:0001",
  "term_label": "Unknown molecular function",
  "gene_symbol": "HSCB",
  "gene": "UniProtKB:Q8IWL3"
}